{
  "gene_symbol": "IGHV3-43D",
  "term_label": "antigen binding",
  "term_id": "GO:0003823",
  "gene": "UniProtKB:P0DP04",
  "gene_name": "Immunoglobulin heavy variable 3-43D"
}